mammary gland involution [GO:0060056] (biological process) Definition: The tissue remodeling that removes differentiated mammary epithelia during weaning. Relationships: is a type of tissue remodeling [GO:0048771]; is part of mammary gland morphogenesis [GO:0060443] References: PMID:15282149 Sources: GOC:dph Regulation: regulated by GO:1903519; negatively regulated by negative regulation of mammary gland involution [GO:1903520]; positively regulated by positive regulation of mammary gland involution [GO:1903521]